regulation of cell adhesion involved in single-species biofilm formation [GO:1900187] (biological process) Definition: Any process that modulates the frequency, rate or extent of cell adhesion involved in single-species biofilm formation. Relationships: is a type of regulation of cell-substrate adhesion [GO:0010810]; regulates cell adhesion involved in single-species biofilm formation [GO:0043709] Subtypes: negative regulation of cell adhesion involved in single-species biofilm formation [GO:1900188], GO:1900189 Also known as: regulation of cell adhesion during single-species biofilm formation Sources: GOC:TermGenie, GOC:di